{
  "gene_symbol": "PRELID3B",
  "term_id": "GO:0005758",
  "gene_name": "PRELI domain containing protein 3B",
  "term_label": "mitochondrial intermembrane space",
  "gene": "UniProtKB:Q9Y3B1"
}